{
  "gene": "UniProtKB:Q9HCK5",
  "term_label": "nucleus",
  "gene_symbol": "AGO4",
  "term_id": "GO:0005634",
  "gene_name": "Protein argonaute-4"
}